{
  "gene": "UniProtKB:P11940",
  "term_id": "GO:1990904",
  "gene_symbol": "PABPC1",
  "gene_name": "Polyadenylate-binding protein 1",
  "term_label": "ribonucleoprotein complex"
}